{
  "gene_symbol": "TJP2",
  "term_id": "GO:0098609",
  "term_label": "cell-cell adhesion",
  "gene_name": "Tight junction protein ZO-2",
  "gene": "UniProtKB:Q9UDY2"
}